lipid storage [GO:0019915] (biological process) Definition: The accumulation and maintenance in cells or tissues of lipids, compounds soluble in organic solvents but insoluble or sparingly soluble in aqueous solvents. Lipid reserves can be accumulated during early developmental stages for mobilization and utilization at later stages of development. Subtypes: cholesterol storage [GO:0010878], triglyceride storage [GO:0030730] Regulation: RO_0002211 by regulation of lipid storage [GO:0010883]; positively regulated by positive regulation of lipid storage [GO:0010884]; negatively regulated by negative regulation of lipid storage [GO:0010888] References: PMID:11102830 Sources: GOC:dph, GOC:mah, GOC:tb Also known as: lipid retention, retention of lipids, sequestration of lipids, storage of lipids, lipid sequestering, lipid sequestration, sequestering of lipids, sequestration of lipid Relationships: is a type of nutrient storage [GO:0170062]